Entner-Doudoroff pathway [GO:0061678] (biological process) Definition: A cellular carbohydrate catabolic process that converts a carbohydrate to pyruvate and either glyceraldehyde or glyceraldehyde-3 phosphate by dehydration and aldol cleavage via a gluconate or 6-phosphogluconate intermediate. Relationships: is a type of GO:0006090; is a type of carbohydrate catabolic process [GO:0016052] Subtypes: Entner-Doudoroff pathway through 6-phosphogluconate [GO:0009255], Entner-Doudoroff pathway through gluconate [GO:0061679] References: PMID:12921536 Sources: GOC:dph